sodium-translocating NADH-quinone reductase complex assembly [GO:0160293] (biological process) Definition: The aggregation, arrangement and bonding together of a set of components to form a sodium-translocating NADH-quinone reductase complex. References: PMID:26644436 Also known as: Na(+)-NQR complex assembly, Na(+)-translocating NADH-quinone reductase complex assembly Relationships: is a type of GO:0065003